nucleocytoplasmic transport [GO:0006913] (biological process) Relationships: is a type of nuclear transport [GO:0051169] Regulation: regulated by GO:0046822; negatively regulated by GO:0046823; positively regulated by positive regulation of nucleocytoplasmic transport [GO:0046824] Also known as: nucleocytoplasmic shuttling Sources: GOC:go_curators Subtypes: nuclear export [GO:0051168], import into nucleus [GO:0051170] Definition: The directed movement of molecules between the nucleus and the cytoplasm. Note: Note that transport through the nuclear pore complex is not transmembrane because the nuclear membrane is a double membrane, and is not traversed.